positive regulation of defense response [GO:0031349] (biological process) Sources: GOC:mah Relationships: is a type of regulation of defense response [GO:0031347]; is a type of positive regulation of response to stimulus [GO:0048584]; positively regulates GO:0006952 Definition: Any process that activates or increases the frequency, rate or extent of a defense response. Also known as: up regulation of defense response, up-regulation of defense response, upregulation of defense response, activation of defense response, stimulation of defense response Subtypes: GO:0002760, positive regulation of cellular defense response [GO:0010186], positive regulation of innate immune response [GO:0045089], positive regulation of inflammatory response [GO:0050729], GO:0070961, positive regulation of defense response to insect [GO:1900367], positive regulation of defense response to bacterium [GO:1900426], GO:1901672, positive regulation of defense response to oomycetes [GO:1902290], positive regulation of xenophagy [GO:1904417], positive regulation of behavioral fear response [GO:2000987]